{
  "term_label": "protein localization to plasma membrane",
  "gene_symbol": "PRAM1",
  "gene_name": "PML-RARA-regulated adapter molecule 1",
  "term_id": "GO:0072659",
  "gene": "UniProtKB:Q96QH2"
}